{
  "gene_symbol": "TRAV38-2DV8",
  "term_label": "immunoglobulin complex",
  "gene_name": "T cell receptor alpha variable 38-2_delta variable 8",
  "term_id": "GO:0019814",
  "gene": "UniProtKB:A0JD32"
}